{
  "gene_symbol": "CCN4",
  "gene": "UniProtKB:O95388",
  "term_id": "GO:0045597",
  "gene_name": "CCN family member 4",
  "term_label": "positive regulation of cell differentiation"
}